{
  "gene_symbol": "PRKAR1B",
  "gene_name": "cAMP-dependent protein kinase type I-beta regulatory subunit",
  "term_id": "GO:0005952",
  "gene": "UniProtKB:P31321",
  "term_label": "cAMP-dependent protein kinase complex"
}